{
  "gene": "UniProtKB:Q8NGG4",
  "term_label": "odorant binding",
  "gene_symbol": "OR8H1",
  "gene_name": "Olfactory receptor 8H1",
  "term_id": "GO:0005549"
}